{
  "gene_symbol": "LMNTD1",
  "gene_name": "Lamin tail domain-containing protein 1",
  "term_label": "nuclear envelope",
  "term_id": "GO:0005635",
  "gene": "UniProtKB:Q8N9Z9"
}